embryonic camera-type eye morphogenesis [GO:0048596] (biological process) Definition: The process in which the anatomical structures of the eye are generated and organized during embryonic development. Also known as: embryonic eye morphogenesis Sources: GOC:jid, GOC:mtg_sensu Relationships: is_a embryonic eye morphogenesis [GO:0048048]; is part of embryonic camera-type eye development [GO:0031076]; is part of camera-type eye morphogenesis [GO:0048593]